{
  "gene": "UniProtKB:P25025",
  "term_id": "GO:0007204",
  "term_label": "positive regulation of cytosolic calcium ion concentration",
  "gene_symbol": "CXCR2",
  "gene_name": "C-X-C chemokine receptor type 2"
}